{
  "gene_name": "CCR4-NOT transcription complex subunit 7",
  "gene_symbol": "CNOT7",
  "gene": "UniProtKB:Q9UIV1",
  "term_id": "GO:0000288",
  "term_label": "nuclear-transcribed mRNA catabolic process, deadenylation-dependent decay"
}